{
  "gene_name": "Ubiquitin carboxyl-terminal hydrolase 17-like protein 20",
  "term_id": "GO:0005634",
  "term_label": "nucleus",
  "gene_symbol": "USP17L20",
  "gene": "UniProtKB:D6RJB6"
}